cytokinin 9-beta-glucosyltransferase activity [GO:0080062] (molecular function) References: PMID:15342621 Sources: KEGG_REACTION:R08369 Definition: Catalysis of the reaction: 6-alkylaminopurine + UDP-D-glucose = 6-alkylamino-9-beta-D-glucosylpurine + H+ + UDP. This reaction is an N-glucosylation event. Relationships: is_a GO:0035251